{
  "term_label": "regulation of cytokine production",
  "term_id": "GO:0001817",
  "gene_name": "Butyrophilin-like protein 3",
  "gene_symbol": "BTNL3",
  "gene": "UniProtKB:Q6UXE8"
}